{
  "term_label": "regulation of transcription by RNA polymerase II",
  "gene_name": "Calmodulin-binding transcription activator 1",
  "term_id": "GO:0006357",
  "gene_symbol": "CAMTA1",
  "gene": "UniProtKB:Q9Y6Y1"
}